positive regulation of fumagillin biosynthetic process [GO:1902092] (biological process) Definition: Any process that activates or increases the frequency, rate or extent of fumagillin biosynthetic process. References: PMID:23488861 Sources: GOC:TermGenie, GOC:di Also known as: activation of fumagillin anabolism, activation of fumagillin biosynthesis, activation of fumagillin formation, activation of fumagillin synthesis, positive regulation of fumagillin anabolism, positive regulation of fumagillin biosynthesis, positive regulation of fumagillin formation, positive regulation of fumagillin synthesis, up regulation of fumagillin anabolism, up regulation of fumagillin biosynthesis, up regulation of fumagillin biosynthetic process, up regulation of fumagillin formation, up regulation of fumagillin synthesis, up-regulation of fumagillin anabolism, up-regulation of fumagillin biosynthesis, up-regulation of fumagillin biosynthetic process, up-regulation of fumagillin formation, up-regulation of fumagillin synthesis, upregulation of fumagillin anabolism, upregulation of fumagillin biosynthesis, upregulation of fumagillin biosynthetic process, upregulation of fumagillin formation, upregulation of fumagillin synthesis, activation of fumagillin biosynthetic process Relationships: is a type of positive regulation of biosynthetic process [GO:0009891]; is a type of positive regulation of small molecule metabolic process [GO:0062013]; is_a GO:1902090; positively regulates GO:1902086